positive regulation of pyocyanine biosynthetic process [GO:0062162] (biological process) Definition: Any process that increases the frequency, rate or extent of a pyocyanine biosynthetic process. References: PMID:28715477 Also known as: positive regulation of pyocyanin biosynthetic process Relationships: is_a positive regulation of biosynthetic process [GO:0009891]; is a type of regulation of pyocyanine biosynthetic process [GO:0062161]; RO_0002213 pyocyanine biosynthetic process [GO:0106220]